{
  "term_label": "Unknown molecular function",
  "gene_symbol": "CCDC200",
  "term_id": "UNKNOWN:0001",
  "gene": "UniProtKB:A0A1B0GVQ3",
  "gene_name": "Coiled-coil domain-containing protein 200"
}